{
  "term_label": "extrinsic component of membrane",
  "gene_name": "Triple functional domain protein",
  "gene_symbol": "TRIO",
  "gene": "UniProtKB:O75962",
  "term_id": "GO:0019898"
}